{
  "term_id": "GO:0006955",
  "term_label": "immune response",
  "gene_name": "C-C chemokine receptor type 10",
  "gene": "UniProtKB:P46092",
  "gene_symbol": "CCR10"
}